transcription initiation at RNA polymerase II promoter [GO:0006367] (biological process) Note: Note that promoter clearance is represented as a separate step, not part_of either initiation or elongation. Definition: A transcription initiation process that takes place at a RNA polymerase II gene promoter. Messenger RNAs (mRNA) genes, as well as some non-coding RNAs, are transcribed by RNA polymerase II. Relationships: is a type of DNA-templated transcription initiation [GO:0006352]; is part of transcription by RNA polymerase II [GO:0006366] Sources: GOC:mah, GOC:txnOH Regulation: RO_0002211 by regulation of transcription initiation by RNA polymerase II [GO:0060260]; positively regulated by positive regulation of transcription initiation by RNA polymerase II [GO:0060261]; negatively regulated by GO:0060633 Also known as: transcription initiation from Pol II promoter, transcription initiation from RNA polymerase II promoter